{
  "term_label": "metallopeptidase activity",
  "gene_symbol": "BRCC3",
  "term_id": "GO:0008237",
  "gene_name": "Lys-63-specific deubiquitinase BRCC36",
  "gene": "UniProtKB:P46736"
}